{
  "gene_symbol": "IL12RB1",
  "gene_name": "Interleukin-12 receptor subunit beta-1",
  "term_label": "cytokine binding",
  "term_id": "GO:0019955",
  "gene": "UniProtKB:P42701"
}